{
  "gene_symbol": "TRAJ38",
  "gene": "UniProtKB:A0A075B6W7",
  "term_id": "UNKNOWN:0003",
  "term_label": "Unknown cellular component",
  "gene_name": "T cell receptor alpha joining 38 (Fragment)"
}